positive regulation of monoatomic anion transport [GO:1903793] (biological process) Also known as: positive regulation of anion transport, up regulation of anion transport, up-regulation of anion transport, upregulation of anion transport, activation of anion transport Definition: Any process that activates or increases the frequency, rate or extent of anion transport. Subtypes: positive regulation of anion transmembrane transport [GO:1903961], positive regulation of iodide transport [GO:1904203] References: PMID:11336802 Sources: GOC:TermGenie, GO_REF:0000058 Relationships: is a type of GO:0043270; is a type of regulation of monoatomic anion transport [GO:0044070]; positively regulates monoatomic anion transport [GO:0006820]